{
  "gene_name": "Cell cycle checkpoint protein RAD17",
  "term_label": "DNA repair",
  "gene": "UniProtKB:O75943",
  "gene_symbol": "RAD17",
  "term_id": "GO:0006281"
}